{
  "term_id": "GO:0098609",
  "gene": "UniProtKB:Q99569",
  "term_label": "cell-cell adhesion",
  "gene_name": "Plakophilin-4",
  "gene_symbol": "PKP4"
}